{
  "term_id": "UNKNOWN:0002",
  "gene": "UniProtKB:Q8NH60",
  "term_label": "Unknown biological process",
  "gene_name": "Olfactory receptor 52J3",
  "gene_symbol": "OR52J3"
}